{
  "gene_name": "Putative protein FAM90A5P",
  "gene": "UniProtKB:A8MXJ8",
  "term_label": "Unknown cellular component",
  "term_id": "UNKNOWN:0003",
  "gene_symbol": "FAM90A5P"
}